monocyte proliferation [GO:0061516] (biological process) Relationships: is a type of leukocyte proliferation [GO:0070661] References: PMID:18467591 Sources: GOC:dph Definition: The expansion of a monocyte population by cell division.